{
  "term_id": "GO:0007010",
  "gene": "UniProtKB:Q9UNF0",
  "gene_symbol": "PACSIN2",
  "gene_name": "Protein kinase C and casein kinase substrate in neurons protein 2",
  "term_label": "cytoskeleton organization"
}